{
  "term_label": "cysteine-type deubiquitinase activity",
  "gene_name": "Ubiquitin carboxyl-terminal hydrolase 7",
  "gene": "UniProtKB:Q93009",
  "term_id": "GO:0004843",
  "gene_symbol": "USP7"
}